minor groove of adenine-thymine-rich DNA binding [GO:0003680] (molecular function) Definition: Binding to a DNA structure formed by the minor groove of adenine-thymine-rich DNA regions. Examples of proteins having this function are AT-rich interaction domain (ARID)-containing proteins. References: PMID:10545119, PMID:15802641, PMID:26223912, PMID:2670564 Sources: GOC:jl Also known as: AT DNA binding, AT binding, AT-rich DNA binding Relationships: is a type of DNA secondary structure binding [GO:0000217]